{
  "gene_symbol": "TRPT1",
  "gene_name": "tRNA 2'-phosphotransferase 1",
  "term_label": "tRNA splicing, via endonucleolytic cleavage and ligation",
  "term_id": "GO:0006388",
  "gene": "UniProtKB:Q86TN4"
}